negative regulation of octopamine signaling pathway involved in response to food [GO:2000140] (biological process) Relationships: is a type of negative regulation of response to food [GO:0032096]; is a type of negative regulation of octopamine signaling pathway [GO:2000129]; is a type of regulation of octopamine signaling pathway involved in response to food [GO:2000139]; negatively regulates octopamine signaling pathway involved in response to food [GO:0071935] References: PMID:19609300 Sources: GOC:mah Also known as: negative regulation of octopamine signalling pathway involved in response to food Definition: Any process that stops, prevents, or reduces the frequency, rate or extent of octopamine signaling pathway involved in response to food.